{
  "term_id": "GO:0005886",
  "gene_name": "12-(S)-hydroxy-5,8,10,14-eicosatetraenoic acid receptor",
  "term_label": "plasma membrane",
  "gene": "UniProtKB:O00270",
  "gene_symbol": "GPR31"
}